oxidoreductase activity, acting on superoxide radicals as acceptor [GO:0016721] (molecular function) Sources: GOC:ai Relationships: is a type of GO:0016491 Definition: Catalysis of an oxidation-reduction (redox) reaction in which a superoxide radical (O2- or O2.-) acts as a hydrogen or electron acceptor. Subtypes: superoxide dismutase activity [GO:0004784], superoxide reductase activity [GO:0050605]